{
  "gene_symbol": "STARD9",
  "term_label": "nucleus",
  "gene_name": "StAR-related lipid transfer protein 9",
  "term_id": "GO:0005634",
  "gene": "UniProtKB:Q9P2P6"
}